{
  "gene_symbol": "SDHD",
  "term_id": "GO:0048039",
  "gene_name": "Succinate dehydrogenase [ubiquinone] cytochrome b small subunit, mitochondrial",
  "term_label": "ubiquinone binding",
  "gene": "UniProtKB:O14521"
}